{
  "gene_name": "IQ domain-containing protein N",
  "term_label": "Unknown cellular component",
  "gene_symbol": "IQCN",
  "term_id": "UNKNOWN:0003",
  "gene": "UniProtKB:Q9H0B3"
}